1,3,6,8-tetrahydroxynaphthalene monooxygenase (quinone-forming) activity [GO:0102634] (molecular function) References: PMID:15701630 Sources: GOC:pz Definition: Catalysis of the reaction: naphthalene-1,3,6,8-tetrol + O2 = flaviolin-2-olate + H2O + H+. Relationships: is a type of oxidoreductase activity, acting on single donors with incorporation of molecular oxygen, incorporation of one atom of oxygen (internal monooxygenases or internal mixed function oxidases) [GO:0016703]